{
  "term_label": "androgen receptor signaling pathway",
  "gene_symbol": "SCGB2A1",
  "gene": "UniProtKB:O75556",
  "gene_name": "Mammaglobin-B",
  "term_id": "GO:0030521"
}